{
  "term_id": "GO:0030336",
  "gene_name": "Serine_threonine-protein kinase 24",
  "term_label": "negative regulation of cell migration",
  "gene_symbol": "STK24",
  "gene": "UniProtKB:Q9Y6E0"
}